{
  "term_id": "GO:0070096",
  "gene": "UniProtKB:Q13505",
  "term_label": "mitochondrial outer membrane translocase complex assembly",
  "gene_name": "Metaxin-1",
  "gene_symbol": "MTX1"
}